{
  "gene_name": "Protein APCDD1",
  "term_label": "negative regulation of Wnt signaling pathway",
  "gene": "UniProtKB:Q8J025",
  "gene_symbol": "APCDD1",
  "term_id": "GO:0030178"
}